{
  "gene": "UniProtKB:P25025",
  "term_label": "external side of plasma membrane",
  "gene_symbol": "CXCR2",
  "term_id": "GO:0009897",
  "gene_name": "C-X-C chemokine receptor type 2"
}